{
  "term_label": "Unknown molecular function",
  "gene": "UniProtKB:Q9Y6E2",
  "term_id": "UNKNOWN:0001",
  "gene_name": "eIF5-mimic protein 1",
  "gene_symbol": "BZW2"
}